{
  "gene_symbol": "CAPS",
  "term_label": "Unknown cellular component",
  "gene_name": "Calcyphosin",
  "term_id": "UNKNOWN:0003",
  "gene": "UniProtKB:Q13938"
}